{
  "gene_symbol": "SLC7A3",
  "gene_name": "Cationic amino acid transporter 3",
  "gene": "UniProtKB:Q8WY07",
  "term_label": "plasma membrane",
  "term_id": "GO:0005886"
}